{
  "gene_symbol": "CD99L2",
  "gene_name": "CD99 antigen-like protein 2",
  "term_label": "Unknown biological process",
  "gene": "UniProtKB:Q8TCZ2",
  "term_id": "UNKNOWN:0002"
}